{
  "gene": "UniProtKB:Q96G91",
  "term_id": "GO:0005886",
  "gene_symbol": "P2RY11",
  "gene_name": "P2Y purinoceptor 11",
  "term_label": "plasma membrane"
}